serine palmitoyltransferase complex [GO:0017059] (cellular component) Definition: A protein complex that catalyses the condensation of L-serine with palmitoyl-CoA to form 3-ketosphinganine, the sphingoid base which is the starting point for all sphingolipids. In bacteria the enzyme is a cytoplasmic homodimer, whereas in eukaryotes the enzyme is a multiprotein complex localised to the endoplasmic reticulum. The eukaryotic complex consists of catalytic components (SPTLC1, SPTLC2 and SPTLC3 in humans; LCB1 and LCB2 in S. cerevisiae) and regulatory components, which include activators (SPTSSA/SPTSSB in humans, TSC3 in S. cerevisiae) and negative regulators (ORMDL1/ORMDL2/ORMDL3 in humans, ORM1/2 in S. cerevisiae ). References: PMID:29863195, PMID:33558761 Relationships: is a type of palmitoyltransferase complex [GO:0002178] Also known as: SPOTS complex, SPT, serine C-palmitoyltransferase complex, serine palmitoyltransferase, Orm1/2, Tsc3 and Sac1 complex